{
  "gene": "UniProtKB:P17021",
  "term_label": "RNA polymerase II cis-regulatory region sequence-specific DNA binding",
  "term_id": "GO:0000978",
  "gene_symbol": "ZNF17",
  "gene_name": "Zinc finger protein 17"
}